checkpoint clamp complex [GO:0030896] (cellular component) Definition: Conserved heterotrimeric complex of PCNA-like proteins that is loaded onto DNA at sites of DNA damage. Relationships: is a type of nuclear protein-containing complex [GO:0140513]; BFO_0000050 GO:0000794 Also known as: CCC, Rad9-Hus1-Rad1 (9-1-1) clamp complex Note: Note that the following subunit names have been used: human RAD9/RAD1/HUS1; S. pombe Rad9/Rad1/Hus1; S. cerevisiae Ddc1p/Rad17p/Mec3p. References: PMID:12531008